lysis of host organelle involved in viral entry into host cell [GO:0039664] (biological process) Definition: The viral-induced lysis of an organelle (endosome, lysosome, or caveosome) that is involved in the uptake of a virus into a host cell. Occurs once the virus is within the organelle, and results in transfer of the viral contents from the organelle compartment into the cytoplasm. Sources: GOC:bf, GOC:jl, UniProtKB-KW:KW-1174, VZ:984 Also known as: viral penetration via lysis of host organellar membrane, viral entry into host cell via endosome membrane lysis, viral entry into host cell via lysis of host organelle membrane, viral membrane-lytic protein Relationships: is a type of viral process [GO:0016032]; is part of GO:0046718; has part disruption of plasma membrane integrity in another organism [GO:0051673] Subtypes: macropinosome lysis involved in viral entry into host cell [GO:0075511], endosome lysis involved in viral entry into host cell [GO:0075514]